{
  "gene": "UniProtKB:Q9H6Y5",
  "term_id": "UNKNOWN:0001",
  "term_label": "Unknown molecular function",
  "gene_name": "PDZ domain-containing protein MAGIX",
  "gene_symbol": "MAGIX"
}